osteoblast development [GO:0002076] (biological process) Definition: The process whose specific outcome is the progression of an osteoblast over time, from its formation to the mature structure. Osteoblast development does not include the steps involved in committing a cranial neural crest cell or an osteoprogenitor cell to an osteoblast fate. An osteoblast is a cell that gives rise to bone. Sources: GOC:dph Relationships: is a type of cell development [GO:0048468]; BFO_0000050 GO:0001649